phosphogluconate dehydrogenase (decarboxylating) activity [GO:0004616] (molecular function) Relationships: is a type of oxidoreductase activity, acting on the CH-OH group of donors, NAD or NADP as acceptor [GO:0016616] Also known as: 6-phosphogluconic dehydrogenase activity, 6-phospho-D-gluconate dehydrogenase activity, 6-phospho-D-gluconate:NADP+ 2-oxidoreductase (decarboxylating), 6-phosphogluconate dehydrogenase (decarboxylating), 6-phosphogluconic carboxylase activity, 6PGD activity, phosphogluconic acid dehydrogenase activity Definition: Catalysis of the reaction: 6-phospho-D-gluconate + NADP+ = D-ribulose 5-phosphate + CO2 + NADPH + H+. Sources: EC:1.1.1.44